{
  "term_label": "mitochondrial inner membrane",
  "term_id": "GO:0005743",
  "gene_symbol": "CHDH",
  "gene": "UniProtKB:Q8NE62",
  "gene_name": "Choline dehydrogenase, mitochondrial"
}